alpha4-beta1 integrin-CD53 complex [GO:0070518] (cellular component) Also known as: ITGA4-ITGB1-CD53 complex Relationships: is a type of plasma membrane protein complex [GO:0098797] References: PMID:8757325 Definition: A protein complex that consists of an alpha4-beta1 integrin complex bound to membrane protein CD53, a member of the tetraspan family.